alpha-L-arabinofuranosidase activity [GO:0046556] (molecular function) Also known as: polysaccharide alpha-L-arabinofuranosidase activity, L-arabinosidase activity, alpha-L-arabinanase activity, alpha-L-arabinofuranoside arabinofuranohydrolase activity, alpha-L-arabinofuranoside hydrolase activity, alpha-L-arabinosidase activity, alpha-N-arabinofuranosidase activity, alpha-arabinofuranosidase activity, alpha-arabinosidase activity, arabinofuranosidase activity, arabinosidase activity Sources: EC:3.2.1.55, GOC:mf Relationships: is a type of GO:0004553 Definition: Catalysis of the hydrolysis of terminal non-reducing alpha-L-arabinofuranoside residues in alpha-L-arabinosides.